peptidyl-cysteine modification [GO:0018198] (biological process) Subtypes: N-terminal peptidyl-L-cysteine N-palmitoylation [GO:0018009], N-terminal protein amino acid deamination, from amino carbon [GO:0018058], peptidyl-L-3-oxoalanine biosynthetic process from peptidyl-cysteine or peptidyl-serine [GO:0018083], GO:0018119, GO:0018125, peptidyl-pyrromethane cofactor linkage [GO:0018160], peptidyl-cysteine oxidation [GO:0018171], peptidyl-S-diacylglycerol-L-cysteine biosynthetic process from peptidyl-cysteine [GO:0018231], peptide cross-linking via L-cystine [GO:0018316], GO:0018339, nickel incorporation into iron-sulfur cluster via tris-L-cysteinyl L-cysteine persulfido L-glutamato L-histidino L-serinyl nickel triiron disulfide trioxide [GO:0018418], peptidyl-cysteine acetylation [GO:0018533], peptidyl-cysteine deglycation [GO:0036526] Relationships: is a type of peptidyl-amino acid modification [GO:0018193] Definition: The modification of peptidyl-cysteine. Sources: GOC:go_curators